{
  "gene_symbol": "FBXO6",
  "term_label": "cytoplasm",
  "term_id": "GO:0005737",
  "gene": "UniProtKB:Q9NRD1",
  "gene_name": "F-box only protein 6"
}